{
  "term_id": "GO:0030308",
  "gene_symbol": "CGRRF1",
  "gene_name": "Cell growth regulator with RING finger domain protein 1",
  "gene": "UniProtKB:Q99675",
  "term_label": "negative regulation of cell growth"
}